mesonephric mesenchyme morphogenesis [GO:0061221] (biological process) Definition: The process in which the anatomical structures of a mesonephric mesenchymal tissue are generated and organized. Mesonephric mesenchyme is the tissue made up of loosely connected mesenchymal cells in the mesonephros. Sources: GOC:mtg_kidney_jan10 Relationships: is a type of kidney mesenchyme morphogenesis [GO:0072131]; is part of mesonephric mesenchyme development [GO:0061219]